{
  "gene_name": "Vegetative cell wall protein gp1-like",
  "gene_symbol": "A0A8I5KYS1",
  "gene": "UniProtKB:A0A8I5KYS1",
  "term_id": "UNKNOWN:0001",
  "term_label": "Unknown molecular function"
}